{
  "term_label": "cell migration",
  "gene_name": "Integrin beta-5",
  "term_id": "GO:0016477",
  "gene_symbol": "ITGB5",
  "gene": "UniProtKB:P18084"
}